{
  "gene": "UniProtKB:Q9H2Y9",
  "gene_name": "Solute carrier organic anion transporter family member 5A1",
  "gene_symbol": "SLCO5A1",
  "term_id": "GO:0043252",
  "term_label": "sodium-independent organic anion transport"
}